positive regulation of transforming growth factor beta production [GO:0071636] (biological process) Sources: GOC:mah Also known as: positive regulation of TGF-B production, positive regulation of TGF-beta production, positive regulation of TGFB production, positive regulation of TGFbeta production, positive regulation of transforming growth factor-beta production, positive regulation of transforming growth factor-beta secretion Definition: Any process that activates or increases the frequency, rate, or extent of production of transforming growth factor-beta. Relationships: is a type of positive regulation of cytokine production [GO:0001819]; is a type of regulation of transforming growth factor beta production [GO:0071634]; positively regulates GO:0071604 Subtypes: positive regulation of transforming growth factor beta1 production [GO:0032914], positive regulation of transforming growth factor beta2 production [GO:0032915], positive regulation of transforming growth factor beta3 production [GO:0032916]